mitochondrial [4Fe-4S] assembly complex [GO:0120510] (cellular component) Relationships: is_a mitochondrial protein-containing complex [GO:0098798]; is a type of GO:1990229 References: PMID:25347204, PMID:29079644, PMID:33711344, PMID:34660592 Also known as: ISA complex, iron-sulfur assembly complex Definition: A protein complex capable of condensing two 2Fe-2S clusters into one 4Fe-4S center in mitochondria. In S. cerevisiae, it consists of Isa1 and Isa2. In humans it consists of ISCA1 and ISCA2. Additional proteins may be present.